UDP-D-xylose:beta-D-glucoside alpha-1,3-D-xylosyltransferase activity [GO:0140563] (molecular function) Relationships: is a type of UDP-xylosyltransferase activity [GO:0035252] References: PMID:30127001 Sources: EC:2.4.2.42, RHEA:56064 Definition: Catalyzes the reaction: UDP-alpha-D-xylose + [protein with EGF-like domain]-3-O-(beta-D-glucosyl)-L-serine = UDP + [protein with EGF-like domain]-3-O-(alpha-D-xylosyl-(1->3)-beta-D-glucosyl)-L-serine.